{
  "gene": "UniProtKB:Q8NEV8",
  "term_label": "Unknown molecular function",
  "gene_name": "Exophilin-5",
  "gene_symbol": "EXPH5",
  "term_id": "UNKNOWN:0001"
}